{
  "gene_name": "Transcription termination factor 3, mitochondrial",
  "term_id": "GO:0045892",
  "gene_symbol": "MTERF3",
  "term_label": "negative regulation of DNA-templated transcription",
  "gene": "UniProtKB:Q96E29"
}